negative regulation of NK T cell proliferation [GO:0051141] (biological process) Definition: Any process that stops, prevents, or reduces the frequency, rate or extent of natural killer T cell proliferation. Also known as: down regulation of NK T cell proliferation, down-regulation of NK T cell proliferation, downregulation of NK T cell proliferation, negative regulation of NK T lymphocyte proliferation, negative regulation of NK T-cell proliferation, negative regulation of NK T-lymphocyte proliferation, negative regulation of NKT cell proliferation, negative regulation of NT cell proliferation, negative regulation of natural T cell proliferation, negative regulation of natural killer T cell proliferation, inhibition of NK T cell proliferation References: PMID:12154375, PMID:9133426 Sources: ISBN:0781735149 Relationships: is_a negative regulation of alpha-beta T cell proliferation [GO:0046642]; is a type of negative regulation of NK T cell activation [GO:0051134]; is a type of regulation of NK T cell proliferation [GO:0051140]; negatively regulates NK T cell proliferation [GO:0001866]